epithelial to mesenchymal transition involved in cardiac fibroblast development [GO:0060940] (BP) Sources: GOC:mtg_heart Definition: A transition where an epicardial cell loses apical/basolateral polarity, severs intercellular adhesive junctions, degrades basement membrane components and becomes a migratory mesenchymal cell that will mature into a cardiac fibroblast. Relationships: is a type of cardiac epithelial to mesenchymal transition [GO:0060317]; is part of epicardium-derived cardiac fibroblast cell development [GO:0060939]